{
  "term_id": "GO:0048013",
  "gene_name": "Ephrin type-B receptor 6",
  "gene": "UniProtKB:O15197",
  "term_label": "ephrin receptor signaling pathway",
  "gene_symbol": "EPHB6"
}